negative regulation of natural killer cell proliferation involved in immune response [GO:0032821] (biological process) Sources: GOC:mah Relationships: is a type of negative regulation of immune effector process [GO:0002698]; is a type of negative regulation of natural killer cell proliferation [GO:0032818]; is a type of regulation of natural killer cell proliferation involved in immune response [GO:0032820]; is a type of GO:0050777; negatively regulates natural killer cell proliferation involved in immune response [GO:0002324] Also known as: inhibition of natural killer cell proliferation during immune response, down regulation of natural killer cell proliferation during immune response, down-regulation of natural killer cell proliferation during immune response, downregulation of natural killer cell proliferation during immune response, negative regulation of NK cell proliferation during immune response, negative regulation of natural killer cell proliferation during immune response Definition: Any process that stops, prevents, or reduces the frequency, rate or extent of natural killer cell proliferation as part of an immune response.